response to leukemia inhibitory factor [GO:1990823] (biological process) Also known as: response to CDF, response to LIF, response to cholinergic differentiation factor Subtypes: cellular response to leukemia inhibitory factor [GO:1990830] Relationships: is a type of GO:0034097 References: PMID:12801913 Definition: Any process that results in a change in state or activity of a cell or an organism (in terms of movement, secretion, enzyme production, gene expression, etc.) as a result of a leukemia inhibitory factor stimulus.